procentriole replication complex [GO:0120099] (cellular component) Definition: A protein complex that acts as a chaperone or scaffold for centriolar proteins during the maturation of the procentriole. Some of its members may become integrated into the growing centriole. Examples are the CPAP(CENPJ)-STIL complex, CEP192-PLK4 complex or CEP152-PLK4 complex in vertebrates. References: PMID:17576815, PMID:18207742, PMID:21059844, PMID:22020124, PMID:24997597 Sources: GOC:bhm Relationships: is a type of protein-containing complex [GO:0032991]; is part of GO:0005737